{
  "term_label": "cullin family protein binding",
  "gene_symbol": "CCDC22",
  "term_id": "GO:0097602",
  "gene": "UniProtKB:O60826",
  "gene_name": "Coiled-coil domain-containing protein 22"
}